interleukin-6 production [GO:0032635] (biological process) Regulation: regulated by GO:0032675; negatively regulated by GO:0032715; positively regulated by GO:0032755 Definition: The appearance of interleukin-6 due to biosynthesis or secretion following a cellular stimulus, resulting in an increase in its intracellular or extracellular levels. Sources: GOC:mah Also known as: IL-6 production, interleukin-6 biosynthetic process, interleukin-6 secretion Relationships: is a type of cytokine production [GO:0001816]